{
  "gene": "UniProtKB:A0A494BZU2",
  "term_id": "UNKNOWN:0002",
  "gene_name": "BLACAT1 overlapping LEMD1 locus",
  "gene_symbol": "BLACAT1",
  "term_label": "Unknown biological process"
}